R7 cell development [GO:0045467] (biological process) Relationships: is a type of compound eye photoreceptor development [GO:0042051]; is part of GO:0045466 Definition: The process whose specific outcome is the progression of the R7 photoreceptor over time, from its formation to the mature structure. The R7 photoreceptor is the last photoreceptor to develop in the ommatidium. References: PMID:11880339